{
  "term_id": "GO:0005634",
  "term_label": "nucleus",
  "gene_symbol": "DIDO1",
  "gene": "UniProtKB:Q9BTC0",
  "gene_name": "Death-inducer obliterator 1"
}